{
  "gene_symbol": "MANSC4",
  "term_id": "GO:0004867",
  "term_label": "serine-type endopeptidase inhibitor activity",
  "gene_name": "MANSC domain-containing protein 4",
  "gene": "UniProtKB:A6NHS7"
}